{
  "term_id": "UNKNOWN:0002",
  "gene": "UniProtKB:P62888",
  "gene_name": "Large ribosomal subunit protein eL30",
  "gene_symbol": "RPL30",
  "term_label": "Unknown biological process"
}